{
  "term_label": "rRNA processing",
  "gene_name": "PIH1 domain-containing protein 1",
  "gene": "UniProtKB:Q9NWS0",
  "gene_symbol": "PIH1D1",
  "term_id": "GO:0006364"
}